{
  "term_id": "GO:0006955",
  "gene_name": "Major histocompatibility complex class I-related gene protein",
  "gene_symbol": "MR1",
  "term_label": "immune response",
  "gene": "UniProtKB:Q95460"
}